{
  "gene_name": "Rho GDP-dissociation inhibitor 2",
  "gene_symbol": "ARHGDIB",
  "term_label": "membrane",
  "term_id": "GO:0016020",
  "gene": "UniProtKB:P52566"
}